{
  "term_label": "cytoplasmic side of plasma membrane",
  "term_id": "GO:0009898",
  "gene": "UniProtKB:Q9Y4K3",
  "gene_name": "TNF receptor-associated factor 6",
  "gene_symbol": "TRAF6"
}